{
  "gene_name": "Protein SSX1",
  "term_label": "Unknown molecular function",
  "gene_symbol": "SSX1",
  "gene": "UniProtKB:Q16384",
  "term_id": "UNKNOWN:0001"
}